{
  "gene": "UniProtKB:Q9H9Y4",
  "gene_symbol": "GPN2",
  "term_id": "UNKNOWN:0003",
  "gene_name": "GPN-loop GTPase 2",
  "term_label": "Unknown cellular component"
}